{
  "gene": "UniProtKB:O43736",
  "term_label": "plasma membrane",
  "gene_symbol": "ITM2A",
  "gene_name": "Integral membrane protein 2A",
  "term_id": "GO:0005886"
}